{
  "term_label": "negative regulation of hippo signaling",
  "gene_name": "LIM domain-containing protein 1",
  "term_id": "GO:0035331",
  "gene": "UniProtKB:Q9UGP4",
  "gene_symbol": "LIMD1"
}